photoreceptor connecting cilium [GO:0032391] (cellular component) Definition: The portion of the photoreceptor cell cilium linking the photoreceptor inner and outer segments. It's considered to be equivalent to the ciliary transition zone. Also known as: photoreceptor cilium References: PMID:15917207, PMID:22653444, PMID:8718680 Sources: GOC:cilia Relationships: is a type of ciliary transition zone [GO:0035869]; is part of GO:0097733